{
  "term_label": "regulation of immune system process",
  "gene_symbol": "CEACAM3",
  "gene_name": "Carcinoembryonic antigen-related cell adhesion molecule 3",
  "term_id": "GO:0002682",
  "gene": "UniProtKB:P40198"
}